{
  "gene_symbol": "TCAP",
  "gene": "UniProtKB:O15273",
  "term_label": "Z disc",
  "term_id": "GO:0030018",
  "gene_name": "Telethonin"
}